{
  "gene": "UniProtKB:Q9NQZ5",
  "term_label": "Unknown biological process",
  "term_id": "UNKNOWN:0002",
  "gene_symbol": "STARD7",
  "gene_name": "StAR-related lipid transfer protein 7, mitochondrial"
}